transcription regulator inhibitor activity [GO:0140416] (molecular function) References: PMID:10652346 Note: Usage guidance: transcription regulator inhibitors bind to a transcription regulator to prevent it from reaching the chromatin. This activity does not occur at the promoter. For activities that do occur at the promoter, consider GO:0001217 ; DNA-binding transcription repressor activity or GO:0003714 ; transcription corepressor activity. An example of a transcription regulator is TCF23 Q7RTU1 is an example of a protein that regulates transcription factors by heterodimerising or binding to DbTFs and prevent DNA binding and their specific genomic binding site where the dbTF would have activated or repressed transcription. Also an example is NFKBIA P25963 which has a different way of regulating transcription factor activity by sequestering the dbTF (complex) in the cytoplasm. Another example is the HSP90 and HSP23 proteins that sequester steroid receptors away from the DNA. Also known as: DNA-binding transcription factor inhibitor activity Definition: A molecular function regulator that inhibits the activity of a transcription regulator via direct binding and/or post-translational modification. Relationships: is a type of molecular function inhibitor activity [GO:0140678]; is part of regulation of gene expression [GO:0010468]; negatively regulates transcription regulator activity [GO:0140110]